growth plate cartilage chondrocyte growth [GO:0003430] (biological process) Sources: GOC:ascb_2009, GOC:dph, GOC:tb Definition: The growth of a growth plate cartilage chondrocyte, where growth contributes to the progression of the chondrocyte over time from one condition to another. Also known as: growth plate cartilage chondrocyte hypertrophy Subtypes: GO:0003432 Relationships: is a type of GO:0003415; is_a developmental growth involved in morphogenesis [GO:0060560]; is part of growth plate cartilage chondrocyte development [GO:0003431]